{
  "term_id": "UNKNOWN:0001",
  "gene": "UniProtKB:Q86X19",
  "gene_symbol": "TMEM17",
  "gene_name": "Transmembrane protein 17",
  "term_label": "Unknown molecular function"
}